Mpp10 complex [GO:0034457] (cellular component) Definition: A protein complex that forms a subcomplex of the 90S preribosome. In S. cerevisiae, it is composed of Mpp10p, Imp3p and Imp4p. References: PMID:17515605 Sources: GOC:mah Note: Note that the term name uses Saccharomyces gene product names because no other names have yet arisen for this complex; the term nevertheless can be used for analogous complexes in other eukaryotes, and the name can be changed if better wording is found. Relationships: is a type of nuclear protein-containing complex [GO:0140513]; is part of nucleolus [GO:0005730]; is part of 90S preribosome [GO:0030686]